{
  "gene": "UniProtKB:P49286",
  "term_id": "GO:0007186",
  "gene_symbol": "MTNR1B",
  "gene_name": "Melatonin receptor type 1B",
  "term_label": "G protein-coupled receptor signaling pathway"
}